{
  "gene_name": "Nck-associated protein 5-like",
  "gene_symbol": "NCKAP5L",
  "term_label": "microtubule plus-end",
  "term_id": "GO:0035371",
  "gene": "UniProtKB:Q9HCH0"
}